termination of RNA polymerase III transcription [GO:0006386] (biological process) Definition: A transcription termination process that completes the production of a primary RNA polymerase II transcript. RNA polymerase III has an intrinsic ability to terminate transcription upon incorporation of at least 4 contiguous U residues. Relationships: is a type of DNA-templated transcription termination [GO:0006353]; is part of transcription by RNA polymerase III [GO:0006383] References: PMID:12944462, PMID:27371117 Sources: GOC:mah Also known as: RNA polymerase III transcription termination, transcription termination from Pol III promoter, transcription termination from RNA polymerase III promoter, RNA polymerase III transcription termination factor activity